negative regulation of immune response [GO:0050777] (BP) Relationships: is a type of negative regulation of immune system process [GO:0002683]; is a type of GO:0048585; is_a regulation of immune response [GO:0050776]; negatively regulates GO:0006955 Subtypes: GO:0002820, GO:0002829, negative regulation of immune response to tumor cell [GO:0002838], GO:0002862, negative regulation of humoral immune response [GO:0002921], GO:0032821, GO:0032827, negative regulation of CD4-positive, CD25-positive, alpha-beta regulatory T cell differentiation involved in immune response [GO:0032833], negative regulation of mast cell activation involved in immune response [GO:0033007], negative regulation of eosinophil degranulation [GO:0043310], GO:0043314, negative regulation of memory T cell differentiation [GO:0043381], GO:0045623, negative regulation of innate immune response [GO:0045824], negative regulation of plasma cell differentiation [GO:1900099], GO:1903582, negative regulation of T cell activation via T cell receptor contact with antigen bound to MHC molecule on antigen presenting cell [GO:2001189], negative regulation of gamma-delta T cell activation involved in immune response [GO:2001192] Sources: GOC:ai Definition: Any process that stops, prevents, or reduces the frequency, rate or extent of the immune response, the immunological reaction of an organism to an immunogenic stimulus. Also known as: down regulation of immune response, down-regulation of immune response, downregulation of immune response, inhibition of immune response